positive regulation of apoptotic process involved in metanephric collecting duct development [GO:1900216] (biological process) References: PMID:17314325 Sources: GOC:TermGenie, GOC:mtg_kidney_jan10, GOC:yaf Definition: Any process that activates or increases the frequency, rate or extent of apoptotic process involved in metanephric collecting duct development. Also known as: activation of apoptotic cell death of metanephric collecting duct development, activation of apoptotic process of metanephric collecting duct development, activation of apoptotic programmed cell death of metanephric collecting duct development, activation of programmed cell death by apoptosis of metanephric collecting duct development, positive regulation of apoptotic cell death of metanephric collecting duct development, positive regulation of apoptotic process of metanephric collecting duct development, positive regulation of apoptotic programmed cell death of metanephric collecting duct development, positive regulation of programmed cell death by apoptosis of metanephric collecting duct development, up regulation of apoptotic cell death of metanephric collecting duct development, up regulation of apoptotic process involved in metanephric collecting duct development, up regulation of apoptotic process of metanephric collecting duct development, up regulation of apoptotic programmed cell death of metanephric collecting duct development, up regulation of programmed cell death by apoptosis of metanephric collecting duct development, up-regulation of apoptotic cell death of metanephric collecting duct development, up-regulation of apoptotic process involved in metanephric collecting duct development, up-regulation of apoptotic process of metanephric collecting duct development, up-regulation of apoptotic programmed cell death of metanephric collecting duct development, up-regulation of programmed cell death by apoptosis of metanephric collecting duct development, upregulation of apoptotic cell death of metanephric collecting duct development, upregulation of apoptotic process involved in metanephric collecting duct development, upregulation of apoptotic process of metanephric collecting duct development, upregulation of apoptotic programmed cell death of metanephric collecting duct development, upregulation of programmed cell death by apoptosis of metanephric collecting duct development, activation of apoptosis of metanephric collecting duct development, activation of apoptotic process involved in metanephric collecting duct development, activation of apoptotic program of metanephric collecting duct development, activation of type I programmed cell death of metanephric collecting duct development, positive regulation of apoptosis of metanephric collecting duct development, positive regulation of apoptotic program of metanephric collecting duct development, positive regulation of type I programmed cell death of metanephric collecting duct development, up regulation of apoptosis of metanephric collecting duct development, up regulation of apoptotic program of metanephric collecting duct development, up regulation of type I programmed cell death of metanephric collecting duct development, up-regulation of apoptosis of metanephric collecting duct development, up-regulation of apoptotic program of metanephric collecting duct development, up-regulation of type I programmed cell death of metanephric collecting duct development, upregulation of apoptosis of metanephric collecting duct development, upregulation of apoptotic program of metanephric collecting duct development, upregulation of type I programmed cell death of metanephric collecting duct development, activation of signaling (initiator) caspase activity of metanephric collecting duct development, positive regulation of signaling (initiator) caspase activity of metanephric collecting duct development, up regulation of signaling (initiator) caspase activity of metanephric collecting duct development, up-regulation of signaling (initiator) caspase activity of metanephric collecting duct development, upregulation of signaling (initiator) caspase activity of metanephric collecting duct development Relationships: is a type of GO:1900214; is a type of positive regulation of apoptotic process involved in development [GO:1904747]; RO_0002213 apoptotic process involved in metanephric collecting duct development [GO:1900204]